{
  "term_label": "adenylate cyclase-activating adrenergic receptor signaling pathway",
  "gene_name": "Beta-2 adrenergic receptor",
  "gene": "UniProtKB:P07550",
  "gene_symbol": "ADRB2",
  "term_id": "GO:0071880"
}